sphingosine beta-galactosyltransferase activity [GO:0047258] (molecular function) Sources: EC:2.4.1.23, RHEA:19485 Relationships: is a type of UDP-galactosyltransferase activity [GO:0035250] Also known as: UDP-galactose:sphingosine 1-beta-galactotransferase activity, UDPgalactose:sphingosine 1-beta-galactotransferase activity, UDPgalactose:sphingosine O-galactosyl transferase activity, galactosyl-sphingosine transferase activity, psychosine-UDP galactosyltransferase activity, psychosine-uridine diphosphate galactosyltransferase activity, uridine diphosphogalactose-sphingosine beta-galactosyltransferase activity Definition: Catalysis of the reaction: sphingosine + UDP-D-galactose = H+ + psychosine + UDP.